positive regulation of glycogen (starch) synthase activity [GO:2000467] (biological process) Definition: Any process that activates or increases the frequency, rate or extent of glycogen (starch) synthase activity. Sources: GOC:obol Also known as: positive regulation of UDP-glucose-glycogen glucosyltransferase activity, positive regulation of UDP-glucose:glycogen 4-alpha-D-glucosyltransferase activity, positive regulation of UDP-glycogen synthase activity, positive regulation of UDPG-glycogen synthetase activity, positive regulation of UDPG-glycogen transglucosylase activity, positive regulation of UDPglucose:glycogen 4-alpha-D-glucosyltransferase activity, positive regulation of glycogen (starch) synthetase activity, positive regulation of uridine diphosphoglucose-glycogen glucosyltransferase activity Relationships: is_a positive regulation of catalytic activity [GO:0043085]; is a type of GO:2000465; positively regulates alpha-1,4-glucan glucosyltransferase (UDP-glucose donor) activity [GO:0004373]